positive regulation of melanin biosynthetic process [GO:0048023] (biological process) Definition: Any process that activates or increases the rate or extent of the chemical reactions and pathways resulting in the formation of melanin. Also known as: positive regulation of melanin anabolism, positive regulation of melanin biosynthesis, positive regulation of melanin formation, positive regulation of melanin synthesis, up regulation of melanin biosynthetic process, up-regulation of melanin biosynthetic process, upregulation of melanin biosynthetic process, activation of melanin biosynthetic process, stimulation of melanin biosynthetic process Sources: GOC:jid Relationships: is a type of regulation of melanin biosynthetic process [GO:0048021]; is a type of positive regulation of secondary metabolite biosynthetic process [GO:1900378]; positively regulates melanin biosynthetic process [GO:0042438]